Tie signaling pathway [GO:0048014] (BP) References: PMID:11283723, PMID:11566266 Sources: GOC:ceb, GOC:signaling Definition: The series of molecular signals initiated by an angiopoietin binding to the Tie receptor, and ending with the regulation of a downstream cellular process, e.g. transcription. Also known as: Tek receptor signaling, Tie receptor signaling pathway, Tie receptor signalling pathway, angiopoietin-Tie signaling pathway, angiopoietin/Tie signaling pathway Relationships: is a type of cell surface receptor protein tyrosine kinase signaling pathway [GO:0007169]